{
  "gene_symbol": "RAB29",
  "gene": "UniProtKB:O14966",
  "term_label": "melanosome organization",
  "gene_name": "Ras-related protein Rab-7L1",
  "term_id": "GO:0032438"
}